{
  "term_label": "Unknown molecular function",
  "term_id": "UNKNOWN:0001",
  "gene_symbol": "SAE1",
  "gene_name": "SUMO-activating enzyme subunit 1",
  "gene": "UniProtKB:Q9UBE0"
}